{
  "term_id": "GO:0005829",
  "gene": "UniProtKB:A6NFH5",
  "term_label": "cytosol",
  "gene_name": "Fatty acid-binding protein 12",
  "gene_symbol": "FABP12"
}